{
  "term_label": "cellular response to lipopolysaccharide",
  "gene_name": "C-X-C motif chemokine 5",
  "gene_symbol": "CXCL5",
  "term_id": "GO:0071222",
  "gene": "UniProtKB:P42830"
}